negative regulation of cortisol secretion [GO:0051463] (biological process) Sources: GOC:ai Relationships: is a type of regulation of cortisol secretion [GO:0051462]; is a type of negative regulation of glucocorticoid secretion [GO:2000850]; negatively regulates cortisol secretion [GO:0043400] Definition: Any process that stops, prevents, or reduces the frequency, rate or extent of the regulated release of cortisol from a cell. Also known as: down regulation of cortisol secretion, down-regulation of cortisol secretion, downregulation of cortisol secretion, inhibition of cortisol secretion